{
  "term_label": "phosphatidylinositol binding",
  "gene": "UniProtKB:A0FGR9",
  "gene_name": "Extended synaptotagmin-3",
  "gene_symbol": "ESYT3",
  "term_id": "GO:0035091"
}